{
  "gene_name": "Helicase SRCAP",
  "term_id": "GO:0016887",
  "gene_symbol": "SRCAP",
  "term_label": "ATP hydrolysis activity",
  "gene": "UniProtKB:Q6ZRS2"
}